regulation of sensory perception [GO:0051931] (biological process) Subtypes: GO:0051930, regulation of sensory perception of sweet taste [GO:1904656], regulation of sensory perception of bitter taste [GO:1904660], regulation of detection of mechanical stimulus involved in sensory perception of touch [GO:1905787] Relationships: is a type of regulation of nervous system process [GO:0031644]; regulates GO:0007600 Definition: Any process that modulates the frequency, rate or extent of sensory perception, the series of events required for an organism to receive a sensory stimulus, convert it to a molecular signal, and recognize and characterize the signal. Sources: GOC:ai